choline metabolic process [GO:0019695] (biological process) Definition: The chemical reactions and pathways involving choline (2-hydroxyethyltrimethylammonium), an amino alcohol that occurs widely in living organisms as a constituent of certain types of phospholipids and in the neurotransmitter acetylcholine. Sources: GOC:jl, ISBN:0192801023 Also known as: choline metabolism Relationships: is a type of GO:0008152 Subtypes: glycine betaine biosynthetic process from choline [GO:0019285], choline biosynthetic process [GO:0042425], GO:0042426